tetracycline transmembrane transport [GO:0015904] (biological process) Definition: The directed movement of tetracycline from one side of a membrane to the other. Tetracycline is a broad spectrum antibiotic that blocks binding of aminoacyl tRNA to the ribosomes of both Gram-positive and Gram-negative organisms (and those of organelles). Sources: GOC:curators Also known as: tetracyclin transport, tetracycline transport Relationships: is a type of organic anion transport [GO:0015711]; is a type of organic hydroxy compound transport [GO:0015850]; is a type of GO:0055085